{
  "term_id": "GO:0035861",
  "term_label": "site of double-strand break",
  "gene": "UniProtKB:Q9BWK5",
  "gene_symbol": "CYREN",
  "gene_name": "Cell cycle regulator of non-homologous end joining"
}